{
  "term_id": "GO:0005737",
  "term_label": "cytoplasm",
  "gene_name": "CUGBP Elav-like family member 2",
  "gene_symbol": "CELF2",
  "gene": "UniProtKB:O95319"
}